nephric duct development [GO:0072176] (BP) Relationships: is a type of GO:0035295; is a type of kidney epithelium development [GO:0072073] Sources: GOC:mtg_kidney_jan10 Subtypes: pronephric duct development [GO:0039022], mesonephric duct development [GO:0072177] Definition: The process whose specific outcome is the progression of a nephric duct over time, from its initial formation to a mature structure. A nephric duct is a tube that drains a primitive kidney.